{
  "term_label": "ribosome",
  "gene": "UniProtKB:Q9BYD1",
  "gene_symbol": "MRPL13",
  "term_id": "GO:0005840",
  "gene_name": "Large ribosomal subunit protein uL13m"
}